{
  "gene": "UniProtKB:Q6UWP2",
  "gene_name": "Dehydrogenase_reductase SDR family member 11",
  "term_label": "Unknown biological process",
  "term_id": "UNKNOWN:0002",
  "gene_symbol": "DHRS11"
}